{
  "gene_symbol": "OR5H1",
  "gene": "UniProtKB:A6NKK0",
  "term_id": "GO:0004984",
  "gene_name": "Olfactory receptor 5H1",
  "term_label": "olfactory receptor activity"
}